{
  "gene_symbol": "TLR3",
  "term_id": "GO:0003725",
  "term_label": "double-stranded RNA binding",
  "gene_name": "Toll-like receptor 3",
  "gene": "UniProtKB:O15455"
}